{
  "term_id": "UNKNOWN:0003",
  "term_label": "Unknown cellular component",
  "gene": "UniProtKB:Q8TAF5",
  "gene_name": "Putative uncharacterized protein LQK1",
  "gene_symbol": "FLVCR1-DT"
}